{
  "term_label": "COP9 signalosome",
  "gene_symbol": "GRAP",
  "gene_name": "GRB2-related adapter protein",
  "gene": "UniProtKB:Q13588",
  "term_id": "GO:0008180"
}